{
  "term_label": "protein tag activity",
  "gene_symbol": "ATG12",
  "gene": "UniProtKB:O94817",
  "gene_name": "Ubiquitin-like protein ATG12",
  "term_id": "GO:0031386"
}